{
  "gene": "UniProtKB:P49703",
  "term_id": "GO:0016192",
  "gene_symbol": "ARL4D",
  "gene_name": "ADP-ribosylation factor-like protein 4D",
  "term_label": "vesicle-mediated transport"
}